{
  "gene": "UniProtKB:Q8N4F7",
  "gene_symbol": "RNF175",
  "gene_name": "RING finger protein 175",
  "term_id": "GO:0005789",
  "term_label": "endoplasmic reticulum membrane"
}